{
  "gene": "UniProtKB:Q9H3N1",
  "term_id": "GO:0015036",
  "term_label": "disulfide oxidoreductase activity",
  "gene_symbol": "TMX1",
  "gene_name": "Thioredoxin-related transmembrane protein 1"
}